protein localization to kinetochore [GO:0034501] (biological process) Subtypes: chromosome passenger complex localization to kinetochore [GO:0072356], GO:0140210, protein localization to kinetochore involved in kinetochore assembly [GO:1903394], Bub1-Bub3 complex localization to kinetochore [GO:1990299] Definition: Any process in which a protein is transported to, or maintained at, the kinetochore. Relationships: is a type of protein localization to chromosome, centromeric region [GO:0071459]; is a type of protein localization to condensed chromosome [GO:1903083] Also known as: protein localisation to kinetochore, condensin localization to kinetochore Regulation: regulated by regulation of protein localization to kinetochore [GO:1905340]; negatively regulated by negative regulation of protein localization to kinetochore [GO:1905341]; positively regulated by positive regulation of protein localization to kinetochore [GO:1905342] Sources: GOC:mah